{
  "gene_symbol": "HR",
  "gene_name": "Lysine-specific demethylase hairless",
  "gene": "UniProtKB:O43593",
  "term_label": "histone H3K9 demethylase activity",
  "term_id": "GO:0032454"
}